{
  "gene": "UniProtKB:Q9BXP5",
  "term_id": "GO:0031053",
  "term_label": "primary miRNA processing",
  "gene_name": "Serrate RNA effector molecule homolog",
  "gene_symbol": "SRRT"
}